{
  "gene_symbol": "SAP30L",
  "term_id": "GO:0003712",
  "term_label": "transcription coregulator activity",
  "gene": "UniProtKB:Q9HAJ7",
  "gene_name": "Histone deacetylase complex subunit SAP30L"
}